{
  "gene_name": "PDZ domain-containing protein GIPC2",
  "term_label": "Unknown molecular function",
  "gene": "UniProtKB:Q8TF65",
  "gene_symbol": "GIPC2",
  "term_id": "UNKNOWN:0001"
}